{
  "gene_name": "Immunoglobulin lambda constant 7",
  "gene_symbol": "IGLC7",
  "term_id": "GO:0016064",
  "gene": "UniProtKB:A0M8Q6",
  "term_label": "immunoglobulin mediated immune response"
}